{
  "term_label": "nucleus",
  "gene_symbol": "LPIN3",
  "gene": "UniProtKB:Q9BQK8",
  "gene_name": "Phosphatidate phosphatase LPIN3",
  "term_id": "GO:0005634"
}